{
  "gene": "UniProtKB:Q9Y572",
  "term_label": "protein kinase activity",
  "gene_symbol": "RIPK3",
  "gene_name": "Receptor-interacting serine_threonine-protein kinase 3",
  "term_id": "GO:0004672"
}